{
  "gene": "UniProtKB:P49593",
  "gene_name": "Protein phosphatase 1F",
  "term_id": "GO:0004722",
  "term_label": "protein serine/threonine phosphatase activity",
  "gene_symbol": "PPM1F"
}